endothelial cell chemotaxis to vascular endothelial growth factor [GO:0090668] (biological process) Regulation: regulated by regulation of endothelial cell chemotaxis to vascular endothelial growth factor [GO:1904857]; negatively regulated by negative regulation of endothelial cell chemotaxis to vascular endothelial growth factor [GO:1904858]; RO_0002213 by GO:1904859 References: PMID:21885851 Sources: GOC:BHF, GOC:BHF_miRNA, GOC:rph Relationships: is a type of cell chemotaxis to vascular endothelial growth factor [GO:0090667] Definition: The directed movement of an endothelial cell in response to the presence of vascular endothelial growth factor (VEGF).